tubulin-tyrosine carboxypeptidase [GO:0106423] (molecular function) Definition: Catalysis of the reaction: C-terminal L-alpha-aminoacyl-L-glutamyl-L-glutamyl-L-tyrosyl-[tubulin] + H2O = C-terminal L-alpha-aminoacyl-L-glutamyl-L-glutamyl-[tubulin] + L-tyrosine. References: PMID:29146869, PMID:35482892 Sources: RHEA:57444 Also known as: tubulinyl-Tyr carboxypeptidase Relationships: is a type of metallocarboxypeptidase activity [GO:0004181]